{
  "term_id": "GO:0005829",
  "gene_symbol": "MAT2A",
  "gene": "UniProtKB:P31153",
  "term_label": "cytosol",
  "gene_name": "S-adenosylmethionine synthase isoform type-2"
}